{
  "term_id": "UNKNOWN:0003",
  "term_label": "Unknown cellular component",
  "gene": "UniProtKB:Q8IVU9",
  "gene_name": "Ciliary-associated calcium-binding coiled-coil protein 1",
  "gene_symbol": "CABCOCO1"
}